uridine catabolic process [GO:0006218] (biological process) Definition: The chemical reactions and pathways resulting in the breakdown of uridine, uracil riboside, a ribonucleoside very widely distributed but occurring almost entirely as phosphoric esters in ribonucleotides and ribonucleic acids. Sources: GOC:go_curators Also known as: uridine breakdown, uridine catabolism, uridine degradation Relationships: is a type of uridine metabolic process [GO:0046108]; is a type of pyrimidine ribonucleoside catabolic process [GO:0046133]